{
  "gene": "UniProtKB:Q92565",
  "term_label": "guanyl-nucleotide exchange factor activity",
  "gene_symbol": "RAPGEF5",
  "gene_name": "Rap guanine nucleotide exchange factor 5",
  "term_id": "GO:0005085"
}